{
  "term_id": "UNKNOWN:0003",
  "gene_name": "Melanoma-derived growth regulatory protein",
  "term_label": "Unknown cellular component",
  "gene": "UniProtKB:Q16674",
  "gene_symbol": "MIA"
}